thromboxane A2 receptor binding [GO:0031870] (molecular function) Also known as: prostanoid TP receptor binding, thromboxane A2 receptor ligand Sources: GOC:mah, GOC:nln Definition: Binding to a thromboxane A2 receptor. Relationships: is a type of prostanoid receptor binding [GO:0031862]